{
  "term_label": "mRNA splicing, via spliceosome",
  "gene": "UniProtKB:P08621",
  "term_id": "GO:0000398",
  "gene_symbol": "SNRNP70",
  "gene_name": "U1 small nuclear ribonucleoprotein 70 kDa"
}